{
  "term_label": "phospholipid efflux",
  "gene": "UniProtKB:Q8IZY2",
  "gene_symbol": "ABCA7",
  "term_id": "GO:0033700",
  "gene_name": "Phospholipid-transporting ATPase ABCA7"
}